sex determination, establishment of X:A ratio [GO:0007540] (biological process) Definition: The developmental process in which an organism senses the number of X chromosomes and autosomes in its genomic complement and responds to it. Relationships: is a type of developmental process involved in reproduction [GO:0003006]; is part of primary sex determination, soma [GO:0007539] References: PMID:20622855 Sources: GOC:isa_complete, GOC:mr, Wikipedia:XY_sex-determination_system